spindle assembly [GO:0051225] (biological process) Subtypes: anastral spindle assembly [GO:0055048], GO:0090306, GO:0090307 Relationships: is_a spindle organization [GO:0007051]; is a type of membraneless organelle assembly [GO:0140694]; is part of GO:0007059 Also known as: bipolar spindle biosynthesis, bipolar spindle formation, spindle biosynthesis, spindle formation Regulation: regulated by regulation of spindle assembly [GO:0090169]; negatively regulated by GO:1905831; RO_0002213 by positive regulation of spindle assembly [GO:1905832] Definition: The aggregation, arrangement and bonding together of a set of components to form the spindle, the array of microtubules and associated molecules that serves to move duplicated chromosomes apart. Sources: GOC:ai, GOC:expert_rg, GOC:mtg_sensu, GOC:tb